{
  "term_label": "piRNA processing",
  "gene": "UniProtKB:Q8N2A8",
  "gene_name": "Mitochondrial cardiolipin hydrolase",
  "gene_symbol": "PLD6",
  "term_id": "GO:0034587"
}